protein myristoylation [GO:0018377] (biological process) Sources: GOC:ai Also known as: protein amino acid myristoylation Relationships: is a type of protein lipidation [GO:0006497]; is a type of protein acylation [GO:0043543] Definition: The covalent attachment of a myristoyl group to a protein. Subtypes: GO:0006499